neural fold formation [GO:0001842] (biological process) Definition: The process in which the neural fold is formed. The edges of the neural plate thicken and move up to form a U-shaped structure called the neural groove. Also known as: neural groove formation Sources: GOC:dph, ISBN:0878932437 Relationships: is a type of morphogenesis of embryonic epithelium [GO:0016331]; is a type of anatomical structure formation involved in morphogenesis [GO:0048646]; is a type of morphogenesis of an epithelial fold [GO:0060571]; is part of primary neural tube formation [GO:0014020]